{
  "term_label": "cellular response to hypoxia",
  "gene_symbol": "EGLN3",
  "gene_name": "Prolyl hydroxylase EGLN3",
  "term_id": "GO:0071456",
  "gene": "UniProtKB:Q9H6Z9"
}